{
  "term_id": "GO:0003724",
  "gene_symbol": "DHX8",
  "gene_name": "ATP-dependent RNA helicase DHX8",
  "term_label": "RNA helicase activity",
  "gene": "UniProtKB:Q14562"
}